{
  "term_label": "plasma membrane",
  "gene": "UniProtKB:Q14833",
  "gene_symbol": "GRM4",
  "gene_name": "Metabotropic glutamate receptor 4",
  "term_id": "GO:0005886"
}